lipid transport across blood-brain barrier [GO:1990379] (biological process) Relationships: is a type of lipid transport [GO:0006869]; is a type of transport across blood-brain barrier [GO:0150104] Also known as: lipid transport across blood brain barrier Definition: The directed movement of lipid molecules passing through the blood-brain barrier. Regulation: regulated by regulation of lipid transport across blood-brain barrier [GO:1903000]; negatively regulated by negative regulation of lipid transport across blood-brain barrier [GO:1903001]; positively regulated by positive regulation of lipid transport across blood-brain barrier [GO:1903002] References: PMID:24345162 Sources: GOC:sjp